positive regulation of removal of superoxide radicals [GO:1904833] (biological process) References: PMID:22836756 Sources: GOC:BHF, GOC:BHF_miRNA, GOC:TermGenie, GOC:rph, GO_REF:0000058 Relationships: is a type of regulation of removal of superoxide radicals [GO:2000121]; is a type of GO:2000379; positively regulates GO:0019430 Definition: Any process that activates or increases the frequency, rate or extent of removal of superoxide radicals. Also known as: positive regulation of cellular detoxification of superoxide radicals, positive regulation of removal of O2-, positive regulation of removal of oxygen free radicals, up regulation of cellular detoxification of superoxide radicals, up regulation of removal of O2-, up regulation of removal of oxygen free radicals, up regulation of removal of superoxide radicals, up-regulation of cellular detoxification of superoxide radicals, up-regulation of removal of O2-, up-regulation of removal of oxygen free radicals, up-regulation of removal of superoxide radicals, upregulation of cellular detoxification of superoxide radicals, upregulation of removal of O2-, upregulation of removal of oxygen free radicals, upregulation of removal of superoxide radicals, activation of cellular detoxification of superoxide radicals, activation of removal of O2-, activation of removal of oxygen free radicals, activation of removal of superoxide radicals